{
  "term_label": "cytoskeletal rearrangement involved in phagocytosis, engulfment",
  "gene_name": "T-cell immunoglobulin and mucin domain-containing protein 4",
  "gene": "UniProtKB:Q96H15",
  "gene_symbol": "TIMD4",
  "term_id": "GO:0060097"
}